ribonucleoside-diphosphate reductase activity, thioredoxin disulfide as acceptor [GO:0004748] (molecular function) Subtypes: ADP reductase activity [GO:0051061], GO:0051062, CDP reductase activity [GO:0051063] Definition: Catalysis of the reaction: 2'-deoxyribonucleoside diphosphate + thioredoxin disulfide + H2O = ribonucleoside diphosphate + thioredoxin. Thioredoxin disulfide is the oxidized form of thioredoxin. Relationships: is a type of ribonucleoside-diphosphate reductase activity [GO:0061731] Also known as: 2'-deoxyribonucleoside-diphosphate:oxidized-thioredoxin 2'-oxidoreductase activity, 2'-deoxyribonucleoside-diphosphate:thioredoxin-disulfide 2'-oxidoreductase activity Sources: EC:1.17.4.1 Note: When thioredoxin is substituted for glutaredoxin in the reaction, annotate instead to 'ribonucleoside-diphosphate reductase, glutaredoxin disulfide as acceptor ; GO:0036175'.